{
  "gene_name": "Angiopoietin-related protein 6",
  "term_label": "extracellular matrix",
  "gene_symbol": "ANGPTL6",
  "gene": "UniProtKB:Q8NI99",
  "term_id": "GO:0031012"
}